{
  "term_label": "innate immune response in mucosa",
  "term_id": "GO:0002227",
  "gene_symbol": "H2BC9",
  "gene_name": "Histone H2B type 1-H",
  "gene": "UniProtKB:Q93079"
}